{
  "gene": "UniProtKB:A6NL46",
  "term_id": "UNKNOWN:0002",
  "gene_symbol": "A6NL46",
  "gene_name": "Putative UPF0607 protein ENSP00000332738",
  "term_label": "Unknown biological process"
}